{
  "gene": "UniProtKB:Q14112",
  "gene_name": "Nidogen-2",
  "gene_symbol": "NID2",
  "term_id": "GO:0005604",
  "term_label": "basement membrane"
}